{
  "gene": "UniProtKB:O15235",
  "term_label": "ribosome",
  "gene_symbol": "MRPS12",
  "term_id": "GO:0005840",
  "gene_name": "Small ribosomal subunit protein uS12m"
}